{
  "term_label": "actin filament organization",
  "gene": "UniProtKB:Q99439",
  "gene_name": "Calponin-2",
  "term_id": "GO:0007015",
  "gene_symbol": "CNN2"
}